{
  "gene_symbol": "TMC1",
  "term_id": "GO:0005245",
  "gene_name": "Transmembrane channel-like protein 1",
  "term_label": "voltage-gated calcium channel activity",
  "gene": "UniProtKB:Q8TDI8"
}